{
  "gene_name": "Putative E3 ubiquitin-protein ligase UBR7",
  "term_id": "UNKNOWN:0003",
  "term_label": "Unknown cellular component",
  "gene_symbol": "UBR7",
  "gene": "UniProtKB:Q8N806"
}